{
  "term_label": "endosome",
  "gene": "UniProtKB:O14525",
  "gene_name": "Astrotactin-1",
  "term_id": "GO:0005768",
  "gene_symbol": "ASTN1"
}